{
  "term_id": "GO:0061891",
  "gene_name": "Synaptotagmin-6",
  "gene_symbol": "SYT6",
  "gene": "UniProtKB:Q5T7P8",
  "term_label": "calcium ion sensor activity"
}